endocrine signaling [GO:0038002] (biological process) Note: This term should be used with caution, and only used when the signaling between cells has been clearly distinguished from paracrine signaling. Sources: GOC:mtg_signaling_feb11, ISBN:0199264678, ISBN:3527303782 Also known as: endocrine signalling Relationships: is a type of GO:0007267; is part of endocrine process [GO:0050886] Definition: The transfer of information from one cell to another, where an endocrine hormone is transported from the signal-producing cell to the receiving cell via the circulatory system (via blood, lymph or cerebrospinal fluid). The signaling cell and the receiving cell are often distant to each other.